{
  "term_label": "nucleus",
  "gene": "UniProtKB:Q6P280",
  "term_id": "GO:0005634",
  "gene_name": "Zinc finger protein 529",
  "gene_symbol": "ZNF529"
}